{
  "term_label": "Unknown cellular component",
  "gene": "UniProtKB:Q9H246",
  "term_id": "UNKNOWN:0003",
  "gene_name": "Uncharacterized protein C1orf21",
  "gene_symbol": "C1orf21"
}